male courtship behavior [GO:0008049] (biological process) Relationships: is a type of courtship behavior [GO:0007619]; is a type of GO:0060179 Definition: The behavior of a male, for the purpose of attracting a sexual partner. An example of this process is found in Drosophila melanogaster. Sources: GOC:mtg_sensu, GOC:pr Subtypes: male courtship behavior, orientation prior to leg tapping and wing vibration [GO:0016543], male courtship behavior, tapping to detect pheromone [GO:0016544], GO:0016546, GO:0045433, male courtship behavior, veined wing extension [GO:0048065] Also known as: male courtship behaviour